{
  "term_label": "BLOC-1 complex",
  "gene": "UniProtKB:Q8TDH9",
  "gene_name": "Biogenesis of lysosome-related organelles complex 1 subunit 5",
  "term_id": "GO:0031083",
  "gene_symbol": "BLOC1S5"
}